chemokine receptor antagonist activity [GO:0046817] (molecular function) Sources: GOC:ai, ISBN:0781718325 Relationships: is a type of receptor antagonist activity [GO:0048019]; is part of GO:0070100 Definition: Interacts with chemokine receptors to reduce the action of a chemokine.